{
  "gene": "UniProtKB:P35606",
  "gene_name": "Coatomer subunit beta'",
  "term_label": "COPI vesicle coat",
  "term_id": "GO:0030126",
  "gene_symbol": "COPB2"
}